{
  "gene_name": "Uncharacterized protein C4orf51",
  "gene_symbol": "C4orf51",
  "term_label": "Unknown molecular function",
  "gene": "UniProtKB:C9J302",
  "term_id": "UNKNOWN:0001"
}